epithelial cell migration involved in metanephric distal tubule morphogenesis [GO:0072291] (biological process) Sources: GOC:mtg_kidney_jan10 Relationships: is a type of GO:0072157; is a type of GO:0072290; is part of metanephric distal tubule morphogenesis [GO:0072287] Definition: The orderly movement of epithelial cells within a renal tubule that contributes to metanephric distal tubule morphogenesis.